{
  "term_label": "Ino80 complex",
  "gene_symbol": "INO80",
  "gene": "UniProtKB:Q9ULG1",
  "term_id": "GO:0031011",
  "gene_name": "Chromatin-remodeling ATPase INO80"
}